{
  "term_id": "GO:1990756",
  "term_label": "ubiquitin-like ligase-substrate adaptor activity",
  "gene_name": "PRAME family member 33",
  "gene": "UniProtKB:A0A0G2JMD5",
  "gene_symbol": "PRAMEF33"
}